{
  "term_label": "extracellular space",
  "gene_symbol": "MANF",
  "gene": "UniProtKB:P55145",
  "term_id": "GO:0005615",
  "gene_name": "Mesencephalic astrocyte-derived neurotrophic factor"
}